positive regulation of establishment of protein localization [GO:1904951] (biological process) Definition: Any process that activates or increases the frequency, rate or extent of establishment of protein localization. Relationships: is a type of positive regulation of biological process [GO:0048518]; is a type of regulation of establishment of protein localization [GO:0070201]; positively regulates establishment of protein localization [GO:0045184] References: PMID:22761445 Sources: GOC:TermGenie, GO_REF:0000058 Subtypes: positive regulation of protein transport [GO:0051222], GO:0090314, positive regulation of establishment of protein localization to mitochondrion [GO:1903749], positive regulation of establishment of protein localization to telomere [GO:1904851] Also known as: positive regulation of establishment of protein localisation, positive regulation of protein positioning, positive regulation of protein recruitment, up regulation of establishment of protein localisation, up regulation of establishment of protein localization, up regulation of protein positioning, up regulation of protein recruitment, up-regulation of establishment of protein localisation, up-regulation of establishment of protein localization, up-regulation of protein positioning, up-regulation of protein recruitment, upregulation of establishment of protein localisation, upregulation of establishment of protein localization, upregulation of protein positioning, upregulation of protein recruitment, activation of establishment of protein localisation, activation of establishment of protein localization, activation of protein positioning, activation of protein recruitment